{
  "gene_name": "Testis-specific basic protein Y 2",
  "term_id": "UNKNOWN:0001",
  "gene_symbol": "BPY2",
  "gene": "UniProtKB:O14599",
  "term_label": "Unknown molecular function"
}